laminaribiose phosphorylase activity [GO:0050045] (molecular function) Relationships: is a type of hexosyltransferase activity [GO:0016758] Sources: EC:2.4.1.31 Definition: Catalysis of the reaction: 3-beta-D-glucosyl-D-glucose + phosphate = D-glucose + alpha-D-glucose 1-phosphate. Also known as: 3-beta-D-glucosyl-D-glucose:phosphate alpha-D-glucosyltransferase activity